nuclear envelope adjacent to nuclear pore complex [GO:0120321] (cellular component) Definition: The region of the nuclear envelope situated in close proximity to a nuclear pore complex. Relationships: is a type of cellular anatomical structure [GO:0110165]; is part of nuclear envelope [GO:0005635] References: PMID:21802294, PMID:24184107 Sources: GOC:mah Also known as: nuclear envelope adjacent to NPC, nuclear envelope periphery of the nuclear pore complex, associated with the nuclear pore